F-9775A catabolic process [GO:1900610] (biological process) Also known as: F-9775A breakdown, F-9775A catabolism, F-9775A degradation Definition: The chemical reactions and pathways resulting in the breakdown of F-9775A. Sources: GOC:TermGenie, GOC:di Relationships: is_a phenol-containing compound catabolic process [GO:0019336]; is a type of polyketide catabolic process [GO:0030640]